cobalt-precorrin-3 C17-methyltransferase activity [GO:0043782] (molecular function) Sources: MetaCyc:RXN-8761 Definition: Catalysis of the reaction: cobalt-precorrin 3 + S-adenosyl-L-methionine = cobalt-precorrin 4 + S-adenosyl-L-homocysteine. Relationships: is a type of methyltransferase activity [GO:0008168] Also known as: cobalt-precorrin-3 methylase, cobalt-precorrin-3 methyltransferase, cobalt-precorrin 3 C17-methyltransferase activity, cobalt-precorrin-3B C17-methyltransferase activity